{
  "gene_symbol": "WDR26",
  "term_label": "proteasome-mediated ubiquitin-dependent protein catabolic process",
  "term_id": "GO:0043161",
  "gene": "UniProtKB:Q9H7D7",
  "gene_name": "WD repeat-containing protein 26"
}